positive regulation of defecation [GO:2000294] (biological process) Subtypes: positive regulation of defecation rhythm [GO:2000748] Definition: Any process that activates or increases the frequency, rate or extent of defecation. Sources: GOC:obol Relationships: is a type of GO:0051047; is a type of GO:0060456; is a type of GO:2000292; positively regulates GO:0030421